{
  "term_id": "GO:0015729",
  "gene_name": "Na(+)_citrate cotransporter",
  "gene": "UniProtKB:Q86YT5",
  "term_label": "oxaloacetate transport",
  "gene_symbol": "SLC13A5"
}